{
  "gene": "UniProtKB:Q8NG11",
  "gene_symbol": "TSPAN14",
  "gene_name": "Tetraspanin-14",
  "term_label": "plasma membrane",
  "term_id": "GO:0005886"
}